{
  "term_id": "UNKNOWN:0002",
  "gene_name": "LRP2-binding protein",
  "gene_symbol": "LRP2BP",
  "term_label": "Unknown biological process",
  "gene": "UniProtKB:Q9P2M1"
}